{
  "term_id": "GO:0007507",
  "gene": "UniProtKB:Q8IX07",
  "gene_name": "Zinc finger protein ZFPM1",
  "term_label": "heart development",
  "gene_symbol": "ZFPM1"
}